ciliary receptor clustering involved in smoothened signaling pathway [GO:0060830] (biological process) Definition: Grouping of smoothened or patched receptors in a cilium, contributing to the smoothened signaling pathway. Sources: GOC:cilia, GOC:dph, GOC:sdb_2009, GOC:tb Also known as: ciliary receptor clustering involved in hedgehog signaling pathway, ciliary receptor clustering involved in hh signaling pathway, ciliary receptor clustering involved in smoothened signalling pathway Relationships: is a type of receptor clustering [GO:0043113]; is part of smoothened signaling pathway [GO:0007224]; occurs in cilium [GO:0005929]